{
  "gene_name": "Arginine-fifty homeobox",
  "term_label": "DNA-binding transcription factor activity, RNA polymerase II-specific",
  "term_id": "GO:0000981",
  "gene": "UniProtKB:A6NJG6",
  "gene_symbol": "ARGFX"
}